myosin I heavy chain binding [GO:0032037] (molecular function) Subtypes: myosin I head/neck binding [GO:0032031], GO:0032032 Sources: GOC:mah Relationships: is a type of myosin I binding [GO:0017024]; is a type of myosin heavy chain binding [GO:0032036] Definition: Binding to a heavy chain of a myosin I complex.